{
  "gene_symbol": "DNPH1",
  "gene": "UniProtKB:O43598",
  "term_label": "5-hydroxymethyl-dUMP N-hydrolase activity",
  "gene_name": "2'-deoxynucleoside 5'-phosphate N-hydrolase 1",
  "term_id": "GO:0070694"
}